adenylate cyclase-activating G protein-coupled receptor signaling pathway [GO:0007189] (biological process) Relationships: is a type of adenylate cyclase-modulating G protein-coupled receptor signaling pathway [GO:0007188]; has part adenylate cyclase activator activity [GO:0010856] Sources: GOC:dph, GOC:mah, GOC:signaling, GOC:tb, ISBN:0815316194 Also known as: G protein signaling, adenylate cyclase activating pathway, G protein signaling, adenylyl cyclase activating pathway, G protein signalling, adenylate cyclase activating pathway, G protein signalling, adenylyl cyclase activating pathway, G-protein signaling, adenylate cyclase activating pathway, G-protein signaling, adenylyl cyclase activating pathway, G-protein signalling, adenylate cyclase activating pathway, G-protein signalling, adenylyl cyclase activating pathway, GPCR signaling pathway via activation of adenylate cyclase, GPCR signaling pathway via activation of adenylate cyclase activity, adenylate cyclase-activating GPCR signaling pathway, positive regulation of adenylate cyclase activity involved in G-protein coupled receptor signaling pathway, activation of adenylate cyclase activity by G-protein signaling pathway, activation of adenylate cyclase activity involved in G-protein signaling, positive regulation of adenylate cyclase activity by G-protein signaling pathway, positive regulation of adenylate cyclase activity by G-protein signalling pathway Subtypes: adenylate cyclase-activating dopamine receptor signaling pathway [GO:0007191], adenylate cyclase-activating serotonin receptor signaling pathway [GO:0007192], GO:0010619, GO:0038035, GO:0038184, adenylate cyclase-activating adrenergic receptor signaling pathway [GO:0071880], adenylate cyclase-activating G protein-coupled cAMP receptor signaling pathway [GO:0140582] Definition: A G protein-coupled receptor signaling pathway in which the signal is transmitted via the activation of adenylyl cyclase activity which results in an increase in the intracellular concentration of cyclic AMP (cAMP). This pathway is negatively regulated by phosphodiesterase, which cleaves cAMP and terminates the signaling. Regulation: regulated by GO:0106070; positively regulated by GO:0106071; RO_0002212 by negative regulation of adenylate cyclase-activating G protein-coupled receptor signaling pathway [GO:0106072] Note: This term can be used to annotate ligands, receptors and G-proteins that lead to activation of adenylate cyclase activity within a signaling pathway.